{
  "term_label": "Unknown cellular component",
  "gene_name": "Immunoglobulin heavy diversity 6-13 (Fragment)",
  "gene_symbol": "IGHD6-13",
  "gene": "UniProtKB:A0A1Y8EI39",
  "term_id": "UNKNOWN:0003"
}